{
  "term_id": "GO:0005737",
  "gene_name": "C-Jun-amino-terminal kinase-interacting protein 2",
  "gene_symbol": "MAPK8IP2",
  "gene": "UniProtKB:Q13387",
  "term_label": "cytoplasm"
}